{
  "gene_name": "Dynein light chain Tctex-type 4",
  "gene_symbol": "DYNLT4",
  "gene": "UniProtKB:Q5JR98",
  "term_label": "dynein intermediate chain binding",
  "term_id": "GO:0045505"
}